{
  "term_id": "UNKNOWN:0002",
  "gene_name": "Fibronectin type III domain-containing protein 8",
  "gene": "UniProtKB:Q8TC99",
  "term_label": "Unknown biological process",
  "gene_symbol": "FNDC8"
}